{
  "gene": "UniProtKB:Q8NG04",
  "term_label": "sulfate transmembrane transporter activity",
  "term_id": "GO:0015116",
  "gene_name": "Putative solute carrier family 26 member 10P",
  "gene_symbol": "SLC26A10P"
}